negative regulation of proteasomal ubiquitin-dependent protein catabolic process [GO:0032435] (biological process) Definition: Any process that stops, prevents, or reduces the frequency, rate or extent of the breakdown of a protein or peptide by hydrolysis of its peptide bonds, initiated by the covalent attachment of ubiquitin, and mediated by the proteasome. Sources: GOC:mah Also known as: down regulation of proteasomal ubiquitin-dependent protein catabolic process, down-regulation of proteasomal ubiquitin-dependent protein catabolic process, downregulation of proteasomal ubiquitin-dependent protein catabolic process, inhibition of proteasomal ubiquitin-dependent protein catabolic process Relationships: is a type of regulation of proteasomal ubiquitin-dependent protein catabolic process [GO:0032434]; is a type of negative regulation of proteasomal protein catabolic process [GO:1901799]; is a type of negative regulation of ubiquitin-dependent protein catabolic process [GO:2000059]; negatively regulates proteasome-mediated ubiquitin-dependent protein catabolic process [GO:0043161] Subtypes: GO:0062026, negative regulation of anaphase-promoting complex-dependent catabolic process [GO:1905785]